{
  "gene": "UniProtKB:Q6AZZ1",
  "gene_name": "E3 ubiquitin-protein ligase TRIM68",
  "gene_symbol": "TRIM68",
  "term_id": "GO:0005654",
  "term_label": "nucleoplasm"
}